{
  "term_label": "Unknown biological process",
  "gene": "UniProtKB:Q9Y3D8",
  "term_id": "UNKNOWN:0002",
  "gene_name": "Adenylate kinase isoenzyme 6",
  "gene_symbol": "AK6"
}